{
  "term_label": "DNA-binding transcription factor activity, RNA polymerase II-specific",
  "gene_name": "Zinc finger Y-chromosomal protein",
  "gene": "UniProtKB:P08048",
  "gene_symbol": "ZFY",
  "term_id": "GO:0000981"
}